{
  "term_label": "U4 snRNA 3'-end processing",
  "gene_symbol": "EXOSC2",
  "term_id": "GO:0034475",
  "gene_name": "Exosome complex component RRP4",
  "gene": "UniProtKB:Q13868"
}